fibrillar collagen trimer [GO:0005583] (cellular component) Relationships: is a type of collagen trimer [GO:0005581]; is part of GO:0098643 Definition: Any triple helical collagen trimer that forms fibrils. Subtypes: GO:0005584, collagen type II trimer [GO:0005585], collagen type III trimer [GO:0005586], collagen type V trimer [GO:0005588], collagen type XI trimer [GO:0005592], GO:1990323, collagen type XXVII trimer [GO:1990325] References: PMID:21421911